{
  "gene": "UniProtKB:Q9C009",
  "term_id": "GO:0000981",
  "gene_name": "Forkhead box protein Q1",
  "term_label": "DNA-binding transcription factor activity, RNA polymerase II-specific",
  "gene_symbol": "FOXQ1"
}